{
  "term_id": "GO:0035556",
  "term_label": "intracellular signal transduction",
  "gene": "UniProtKB:Q92918",
  "gene_name": "Mitogen-activated protein kinase kinase kinase kinase 1",
  "gene_symbol": "MAP4K1"
}